{
  "term_id": "GO:0003735",
  "gene_symbol": "RPL7L1",
  "term_label": "structural constituent of ribosome",
  "gene_name": "Ribosomal protein uL30-like",
  "gene": "UniProtKB:Q6DKI1"
}